{
  "term_id": "UNKNOWN:0001",
  "term_label": "Unknown molecular function",
  "gene_name": "Signal transducing adapter molecule 1",
  "gene": "UniProtKB:Q92783",
  "gene_symbol": "STAM"
}